{
  "term_label": "neuropilin binding",
  "gene": "UniProtKB:Q13275",
  "gene_symbol": "SEMA3F",
  "term_id": "GO:0038191",
  "gene_name": "Semaphorin-3F"
}